{
  "gene_symbol": "PPP4R1",
  "term_label": "protein phosphatase regulator activity",
  "gene": "UniProtKB:Q8TF05",
  "gene_name": "Serine_threonine-protein phosphatase 4 regulatory subunit 1",
  "term_id": "GO:0019888"
}